{
  "term_label": "chromatin remodeling",
  "gene_name": "Nucleoplasmin-3",
  "term_id": "GO:0006338",
  "gene": "UniProtKB:O75607",
  "gene_symbol": "NPM3"
}